{
  "gene_symbol": "SLC15A2",
  "gene_name": "Solute carrier family 15 member 2",
  "term_id": "GO:0140206",
  "gene": "UniProtKB:Q16348",
  "term_label": "dipeptide import across plasma membrane"
}